{
  "gene": "UniProtKB:Q86U38",
  "gene_symbol": "NOP9",
  "gene_name": "Nucleolar protein 9",
  "term_id": "GO:0005730",
  "term_label": "nucleolus"
}